{
  "gene_symbol": "AXL",
  "gene": "UniProtKB:P30530",
  "term_label": "nervous system development",
  "term_id": "GO:0007399",
  "gene_name": "Tyrosine-protein kinase receptor UFO"
}